{
  "gene": "UniProtKB:Q9UHD9",
  "gene_name": "Ubiquilin-2",
  "gene_symbol": "UBQLN2",
  "term_id": "GO:0016241",
  "term_label": "regulation of macroautophagy"
}